{
  "term_label": "myosin V binding",
  "gene_name": "Ras-related protein Rab-10",
  "term_id": "GO:0031489",
  "gene": "UniProtKB:P61026",
  "gene_symbol": "RAB10"
}